{
  "term_label": "neuron projection development",
  "gene_symbol": "VAPA",
  "term_id": "GO:0031175",
  "gene_name": "Vesicle-associated membrane protein-associated protein A",
  "gene": "UniProtKB:Q9P0L0"
}